{
  "term_label": "mitochondrion",
  "gene_symbol": "DHFR2",
  "term_id": "GO:0005739",
  "gene": "UniProtKB:Q86XF0",
  "gene_name": "Dihydrofolate reductase 2, mitochondrial"
}